negative regulation of histidine biosynthetic process [GO:0120214] (biological process) Definition: Any process that stops, prevents or reduces the frequency, rate or extent of histidine biosynthetic process. Also known as: down regulation of histidine anabolism, down regulation of histidine biosynthesis, down regulation of histidine biosynthetic process, down regulation of histidine formation, down regulation of histidine synthesis, down-regulation of histidine anabolism, down-regulation of histidine biosynthesis, down-regulation of histidine biosynthetic process, down-regulation of histidine formation, down-regulation of histidine synthesis, downregulation of histidine anabolism, downregulation of histidine biosynthesis, downregulation of histidine biosynthetic process, downregulation of histidine formation, downregulation of histidine synthesis, negative regulation of histidine anabolism, negative regulation of histidine biosynthesis, negative regulation of histidine formation, negative regulation of histidine synthesis, inhibition of histidine anabolism, inhibition of histidine biosynthesis, inhibition of histidine biosynthetic process, inhibition of histidine formation, inhibition of histidine synthesis Sources: GOC:krc Relationships: is a type of negative regulation of small molecule metabolic process [GO:0062014]; is a type of regulation of histidine biosynthetic process [GO:0120213]; is_a negative regulation of amino acid biosynthetic process [GO:2000283]; negatively regulates GO:0000105